generation of mature 3'-end of 5S rRNA generated by RNA polymerase III [GO:0002107] (biological process) References: PMID:16387655, PMID:1748637, PMID:1902221, PMID:8389357 Sources: GOC:hjd Definition: The removal of extra uridine residues from the 3' end of a 5S pre-rRNA generated by transcription by RNA polymerase III to generate the mature 3'-end. Relationships: is a type of maturation of 5S rRNA [GO:0000481]; is a type of rRNA 3'-end processing [GO:0031125]